{
  "gene_symbol": "FGF21",
  "term_label": "extracellular space",
  "gene_name": "Fibroblast growth factor 21",
  "gene": "UniProtKB:Q9NSA1",
  "term_id": "GO:0005615"
}